zonula adherens maintenance [GO:0045218] (biological process) Definition: Maintaining the zonula adherens junction, the cell-cell adherens junction formed near the apex of epithelial cells. Sources: GOC:bf Relationships: is a type of adherens junction maintenance [GO:0034334]